negative regulation of activated CD8-positive, alpha-beta T cell apoptotic process [GO:1905403] (biological process) References: PMID:24187568 Sources: GOC:TermGenie, GO_REF:0000058 Also known as: down regulation of activated CD8-positive, alpha-beta T cell apoptotic process, down regulation of activated CD8-positive, alpha-beta T lymphocyte apoptotic process, down regulation of activated CD8-positive, alpha-beta T-cell apoptotic process, down regulation of activated CD8-positive, alpha-beta T-lymphocyte apoptotic process, down-regulation of activated CD8-positive, alpha-beta T cell apoptotic process, down-regulation of activated CD8-positive, alpha-beta T lymphocyte apoptotic process, down-regulation of activated CD8-positive, alpha-beta T-cell apoptotic process, down-regulation of activated CD8-positive, alpha-beta T-lymphocyte apoptotic process, downregulation of activated CD8-positive, alpha-beta T cell apoptotic process, downregulation of activated CD8-positive, alpha-beta T lymphocyte apoptotic process, downregulation of activated CD8-positive, alpha-beta T-cell apoptotic process, downregulation of activated CD8-positive, alpha-beta T-lymphocyte apoptotic process, negative regulation of activated CD8-positive, alpha-beta T lymphocyte apoptotic process, negative regulation of activated CD8-positive, alpha-beta T-cell apoptotic process, negative regulation of activated CD8-positive, alpha-beta T-lymphocyte apoptotic process, down regulation of activated CD8-positive, alpha-beta T cell apoptosis, down regulation of activated CD8-positive, alpha-beta T lymphocyte apoptosis, down regulation of activated CD8-positive, alpha-beta T-cell apoptosis, down regulation of activated CD8-positive, alpha-beta T-lymphocyte apoptosis, down-regulation of activated CD8-positive, alpha-beta T cell apoptosis, down-regulation of activated CD8-positive, alpha-beta T lymphocyte apoptosis, down-regulation of activated CD8-positive, alpha-beta T-cell apoptosis, down-regulation of activated CD8-positive, alpha-beta T-lymphocyte apoptosis, downregulation of activated CD8-positive, alpha-beta T cell apoptosis, downregulation of activated CD8-positive, alpha-beta T lymphocyte apoptosis, downregulation of activated CD8-positive, alpha-beta T-cell apoptosis, downregulation of activated CD8-positive, alpha-beta T-lymphocyte apoptosis, inhibition of activated CD8-positive, alpha-beta T cell apoptosis, inhibition of activated CD8-positive, alpha-beta T cell apoptotic process, inhibition of activated CD8-positive, alpha-beta T lymphocyte apoptosis, inhibition of activated CD8-positive, alpha-beta T lymphocyte apoptotic process, inhibition of activated CD8-positive, alpha-beta T-cell apoptosis, inhibition of activated CD8-positive, alpha-beta T-cell apoptotic process, inhibition of activated CD8-positive, alpha-beta T-lymphocyte apoptosis, inhibition of activated CD8-positive, alpha-beta T-lymphocyte apoptotic process, negative regulation of activated CD8-positive, alpha-beta T cell apoptosis, negative regulation of activated CD8-positive, alpha-beta T lymphocyte apoptosis, negative regulation of activated CD8-positive, alpha-beta T-cell apoptosis, negative regulation of activated CD8-positive, alpha-beta T-lymphocyte apoptosis Relationships: is a type of negative regulation of T cell apoptotic process [GO:0070233]; is a type of GO:1905402; negatively regulates GO:1905397 Definition: Any process that stops, prevents or reduces the frequency, rate or extent of activated CD8-positive, alpha-beta T cell apoptotic process.